compound eye cone cell differentiation [GO:0042675] (biological process) Sources: GOC:mtg_sensu Definition: The process in which a relatively unspecialized cell acquires the specialized features of a compound eye cone cell, a cone-shaped cell, that focuses light in a compound eye. Relationships: is a type of cell differentiation [GO:0030154]; is part of GO:0001745